exogenous protein binding [GO:0140272] (MF) Definition: Binding to a protein or protein complex from a different species, for example a pathogen molecule binding to a host protein. References: PMID:28861068 Note: Note that as GO captures normal processes, it may be that exogenous proteins interactions are normal for one of the participating species but not the other. Therefore reciprocal annotations should not be made without confirming that it is physiological relevant. Relationships: is a type of protein binding [GO:0005515] Subtypes: virus receptor activity [GO:0001618], virus coreceptor activity [GO:0120274]